{
  "gene": "UniProtKB:Q96S95",
  "term_id": "GO:0008427",
  "term_label": "calcium-dependent protein kinase inhibitor activity",
  "gene_symbol": "CAMK2N2",
  "gene_name": "Calcium_calmodulin-dependent protein kinase II inhibitor 2"
}